{
  "term_label": "DNA-binding transcription factor activity, RNA polymerase II-specific",
  "term_id": "GO:0000981",
  "gene_symbol": "ZNF844",
  "gene_name": "Zinc finger protein 844",
  "gene": "UniProtKB:Q08AG5"
}